{
  "term_label": "Unknown biological process",
  "term_id": "UNKNOWN:0002",
  "gene_symbol": "MSRB2",
  "gene_name": "Methionine-R-sulfoxide reductase B2, mitochondrial",
  "gene": "UniProtKB:Q9Y3D2"
}